{
  "gene_name": "Collagen alpha-2(XI) chain",
  "gene": "UniProtKB:P13942",
  "term_label": "extracellular matrix",
  "gene_symbol": "COL11A2",
  "term_id": "GO:0031012"
}